{
  "term_id": "GO:0005634",
  "term_label": "nucleus",
  "gene_symbol": "CDK2AP1",
  "gene_name": "Cyclin-dependent kinase 2-associated protein 1",
  "gene": "UniProtKB:O14519"
}